G-protein alpha(o)-synembrin complex [GO:0071153] (cellular component) References: PMID:12509430 Sources: GOC:mah Definition: A protein complex formed by the association of the guanine nucleotide exchange factor synembrin with the alpha(o) subunit of a heterotrimeric G protein. Relationships: is a type of intracellular protein-containing complex [GO:0140535]; is part of intracellular anatomical structure [GO:0005622] Also known as: Ric-8A G(o) alpha-1 subunit complex, Ric-8A G(o) alpha-2 subunit complex